{
  "term_label": "Cul3-RING ubiquitin ligase complex",
  "gene_name": "Kelch repeat and BTB domain-containing protein 3",
  "term_id": "GO:0031463",
  "gene_symbol": "KBTBD3",
  "gene": "UniProtKB:Q8NAB2"
}